{
  "gene_symbol": "MAT2A",
  "gene": "UniProtKB:P31153",
  "term_id": "GO:0048269",
  "gene_name": "S-adenosylmethionine synthase isoform type-2",
  "term_label": "methionine adenosyltransferase complex"
}